regulation of granzyme B production [GO:0071661] (biological process) Subtypes: negative regulation of granzyme B production [GO:0071662], positive regulation of granzyme B production [GO:0071663] Sources: GOC:mah Relationships: is a type of GO:0001817; is a type of regulation of production of molecular mediator of immune response [GO:0002700]; regulates granzyme B production [GO:0071613] Definition: Any process that modulates the frequency, rate, or extent of production of granzyme B.